{
  "term_label": "positive regulation of T cell receptor signaling pathway",
  "gene_symbol": "NECTIN2",
  "term_id": "GO:0050862",
  "gene_name": "Nectin-2",
  "gene": "UniProtKB:Q92692"
}